{
  "gene_symbol": "DOCK11",
  "term_id": "GO:0051491",
  "gene": "UniProtKB:Q5JSL3",
  "term_label": "positive regulation of filopodium assembly",
  "gene_name": "Dedicator of cytokinesis protein 11"
}